satellite cell activation involved in skeletal muscle regeneration [GO:0014901] (biological process) Regulation: regulated by GO:0014717; positively regulated by positive regulation of satellite cell activation involved in skeletal muscle regeneration [GO:0014718]; negatively regulated by negative regulation of skeletal muscle satellite cell activation involved in skeletal muscle regeneration [GO:1901667] Sources: GOC:mtg_muscle Relationships: is a type of skeletal muscle satellite cell activation [GO:0014719]; is part of skeletal muscle tissue regeneration [GO:0043403] Definition: The process that initiates skeletal muscle satellite cell division by causing it to move from quiescence to the G1 stage of the cell cycle. The cell swells and there are a number of other small changes. The cells then start to divide. Following cell division the cells will differentiate. In adult muscle, satellite cells become activated to divide and differentiate in response to muscle damage.